{
  "gene_name": "Syndecan-3",
  "gene": "UniProtKB:O75056",
  "term_label": "cell surface",
  "gene_symbol": "SDC3",
  "term_id": "GO:0009986"
}